positive regulation of blood pressure by epinephrine-norepinephrine [GO:0003321] (biological process) Relationships: is a type of regulation of systemic arterial blood pressure by norepinephrine-epinephrine [GO:0001993]; is a type of positive regulation of blood pressure [GO:0045777] Definition: Any process in which the force of blood traveling through the circulatory system is increased by the chemicals epinephrine and norepinephrine. Sources: GOC:dph